{
  "gene_symbol": "PLCB2",
  "gene_name": "1-phosphatidylinositol 4,5-bisphosphate phosphodiesterase beta-2",
  "term_id": "GO:0051209",
  "term_label": "release of sequestered calcium ion into cytosol",
  "gene": "UniProtKB:Q00722"
}